neutral, basic amino acid:sodium:chloride symporter activity [GO:0015374] (molecular function) Also known as: neutral, cationic amino acid:sodium:chloride symporter activity Sources: TC:2.A.22.2.3 Relationships: is a type of GO:0005283; is part of GO:0006821 Definition: Enables the transfer of a solute or solutes from one side of a membrane to the other according to the reaction: neutral/basic amino acid(out) + Na+(out) + Cl-(out) = neutral/basic amino acid(in) + Na+(in) + Cl-(in).